{
  "term_label": "Unknown molecular function",
  "gene_name": "T cell receptor beta variable 11-1",
  "term_id": "UNKNOWN:0001",
  "gene": "UniProtKB:A0A0K0K1C0",
  "gene_symbol": "TRBV11-1"
}